{
  "gene_symbol": "SLA2",
  "term_label": "Unknown cellular component",
  "term_id": "UNKNOWN:0003",
  "gene_name": "Src-like-adapter 2",
  "gene": "UniProtKB:Q9H6Q3"
}